{
  "gene_name": "Sorting nexin-11",
  "term_id": "GO:0016050",
  "gene": "UniProtKB:Q9Y5W9",
  "gene_symbol": "SNX11",
  "term_label": "vesicle organization"
}